{
  "gene": "UniProtKB:Q9UBD3",
  "gene_symbol": "XCL2",
  "gene_name": "Cytokine SCM-1 beta",
  "term_id": "GO:0048020",
  "term_label": "CCR chemokine receptor binding"
}